{
  "gene_symbol": "ZCCHC7",
  "gene": "UniProtKB:Q8N3Z6",
  "term_id": "GO:0071036",
  "gene_name": "Zinc finger CCHC domain-containing protein 7",
  "term_label": "nuclear polyadenylation-dependent snoRNA catabolic process"
}